{
  "gene_name": "CAAX prenyl protease 2",
  "gene_symbol": "RCE1",
  "term_label": "endoplasmic reticulum membrane",
  "gene": "UniProtKB:Q9Y256",
  "term_id": "GO:0005789"
}